hormone catabolic process [GO:0042447] (biological process) Subtypes: GO:0006710, estrogen catabolic process [GO:0006711], mineralocorticoid catabolic process [GO:0006712], GO:0006719, C21-steroid hormone catabolic process [GO:0008208], GO:0009823, GO:0009852, calcitonin catabolic process [GO:0010816], brassinosteroid catabolic process [GO:0016133], GO:0042404, melatonin catabolic process [GO:0042442], pheromone catabolic process [GO:0042812], ecdysteroid catabolic process [GO:0046344] Definition: The chemical reactions and pathways resulting in the breakdown of any hormone, naturally occurring substances secreted by specialized cells that affects the metabolism or behavior of other cells possessing functional receptors for the hormone. Relationships: is a type of catabolic process [GO:0009056]; is a type of hormone metabolic process [GO:0042445] Also known as: hormone breakdown, hormone catabolism, hormone degradation Sources: GOC:jl